{
  "term_id": "GO:0000978",
  "gene_name": "Zinc finger protein ZIC 4",
  "term_label": "RNA polymerase II cis-regulatory region sequence-specific DNA binding",
  "gene_symbol": "ZIC4",
  "gene": "UniProtKB:Q8N9L1"
}